{
  "term_label": "Unknown molecular function",
  "term_id": "UNKNOWN:0001",
  "gene_name": "Caskin-1",
  "gene_symbol": "CASKIN1",
  "gene": "UniProtKB:Q8WXD9"
}